positive regulation of photosynthesis [GO:1905157] (biological process) Definition: Any process that activates or increases the frequency, rate or extent of photosynthesis. Also known as: up regulation of photosynthesis, up-regulation of photosynthesis, upregulation of photosynthesis, activation of photosynthesis References: PMID:7592491 Sources: GOC:TermGenie, GO_REF:0000058 Relationships: is a type of GO:0009893; is a type of regulation of photosynthesis [GO:0010109]; positively regulates photosynthesis [GO:0015979]